{
  "gene": "UniProtKB:P09341",
  "gene_symbol": "CXCL1",
  "term_id": "UNKNOWN:0002",
  "term_label": "Unknown biological process",
  "gene_name": "Growth-regulated alpha protein"
}